{
  "gene_name": "26S proteasome non-ATPase regulatory subunit 4",
  "term_id": "GO:0005634",
  "gene": "UniProtKB:P55036",
  "gene_symbol": "PSMD4",
  "term_label": "nucleus"
}